telomerase catalytic core complex assembly [GO:1904868] (biological process) Also known as: telomerase catalytic core complex formation, TERT-TERC complex assembly, TERT-TERC complex formation Relationships: is a type of telomerase holoenzyme complex assembly [GO:1905323] References: PMID:26586433 Sources: GOC:BHF, GOC:BHF_telomere, GOC:TermGenie, GOC:rph, GO_REF:0000079 Regulation: regulated by regulation of telomerase catalytic core complex assembly [GO:1904882]; negatively regulated by GO:1904883; positively regulated by positive regulation of telomerase catalytic core complex assembly [GO:1904884] Definition: The aggregation, arrangement and bonding together of a set of components to form a telomerase catalytic core complex.